{
  "gene_name": "Mediator of DNA damage checkpoint protein 1",
  "term_id": "GO:0035861",
  "gene": "UniProtKB:Q14676",
  "term_label": "site of double-strand break",
  "gene_symbol": "MDC1"
}